{
  "term_id": "GO:0046624",
  "gene": "UniProtKB:A6NFX1",
  "gene_symbol": "MFSD2B",
  "gene_name": "Sphingosine-1-phosphate transporter MFSD2B",
  "term_label": "sphingolipid transporter activity"
}